{
  "gene_name": "Tumor necrosis factor ligand superfamily member 18",
  "term_id": "GO:0002309",
  "gene_symbol": "TNFSF18",
  "gene": "UniProtKB:Q9UNG2",
  "term_label": "T cell proliferation involved in immune response"
}